{
  "term_id": "GO:0006094",
  "term_label": "gluconeogenesis",
  "gene": "UniProtKB:P35558",
  "gene_name": "Phosphoenolpyruvate carboxykinase, cytosolic [GTP]",
  "gene_symbol": "PCK1"
}